{
  "term_label": "Unknown cellular component",
  "gene_symbol": "OR8U3",
  "term_id": "UNKNOWN:0003",
  "gene": "UniProtKB:Q8NH85",
  "gene_name": "Olfactory receptor 8U3"
}